{
  "term_id": "GO:0006493",
  "gene": "UniProtKB:Q8N4A0",
  "gene_symbol": "GALNT4",
  "gene_name": "Polypeptide N-acetylgalactosaminyltransferase 4",
  "term_label": "protein O-linked glycosylation"
}